{
  "gene_name": "Exportin-1",
  "term_id": "GO:0005049",
  "term_label": "nuclear export signal receptor activity",
  "gene_symbol": "XPO1",
  "gene": "UniProtKB:O14980"
}